positive regulation of antigen processing and presentation of peptide or polysaccharide antigen via MHC class II [GO:0002582] (biological process) Also known as: positive regulation of peptide or polysaccharide antigen processing and presentation via MHC class II, up regulation of antigen processing and presentation of peptide or polysaccharide antigen via MHC class II, up-regulation of antigen processing and presentation of peptide or polysaccharide antigen via MHC class II, upregulation of antigen processing and presentation of peptide or polysaccharide antigen via MHC class II, activation of antigen processing and presentation of peptide or polysaccharide antigen via MHC class II, stimulation of antigen processing and presentation of peptide or polysaccharide antigen via MHC class II Sources: GOC:add Relationships: is_a positive regulation of antigen processing and presentation [GO:0002579]; is a type of regulation of antigen processing and presentation of peptide or polysaccharide antigen via MHC class II [GO:0002580]; positively regulates antigen processing and presentation of peptide or polysaccharide antigen via MHC class II [GO:0002504] Subtypes: positive regulation of antigen processing and presentation of peptide antigen via MHC class II [GO:0002588], positive regulation of antigen processing and presentation of polysaccharide antigen via MHC class II [GO:0002603] Definition: Any process that activates or increases the frequency, rate, or extent of antigen processing and presentation of antigen (peptide or polysaccharide) via MHC class II.